{
  "term_label": "plasma membrane",
  "gene": "UniProtKB:Q92847",
  "gene_symbol": "GHSR",
  "gene_name": "Growth hormone secretagogue receptor type 1",
  "term_id": "GO:0005886"
}